{
  "term_id": "GO:0007165",
  "gene_symbol": "PTPRR",
  "gene": "UniProtKB:Q15256",
  "gene_name": "Receptor-type tyrosine-protein phosphatase R",
  "term_label": "signal transduction"
}